{
  "term_id": "GO:0061630",
  "gene_name": "E3 ubiquitin-protein ligase RNF14",
  "term_label": "ubiquitin protein ligase activity",
  "gene": "UniProtKB:Q9UBS8",
  "gene_symbol": "RNF14"
}